{
  "gene_name": "Protocadherin gamma-B7",
  "gene_symbol": "PCDHGB7",
  "term_id": "GO:0050839",
  "gene": "UniProtKB:Q9Y5F8",
  "term_label": "cell adhesion molecule binding"
}